{
  "term_id": "GO:1902004",
  "gene": "UniProtKB:A4D1B5",
  "term_label": "positive regulation of amyloid-beta formation",
  "gene_symbol": "GSAP",
  "gene_name": "Gamma-secretase-activating protein"
}